{
  "gene_name": "Disks large homolog 2",
  "term_label": "receptor localization to synapse",
  "gene": "UniProtKB:Q15700",
  "term_id": "GO:0097120",
  "gene_symbol": "DLG2"
}